{
  "term_label": "rRNA processing",
  "term_id": "GO:0006364",
  "gene_name": "WD repeat-containing protein 36",
  "gene_symbol": "WDR36",
  "gene": "UniProtKB:Q8NI36"
}